{
  "gene_name": "TLC domain-containing protein 3A",
  "gene": "UniProtKB:Q8TBR7",
  "term_id": "GO:0005783",
  "term_label": "endoplasmic reticulum",
  "gene_symbol": "TLCD3A"
}